mitotic prophase [GO:0000088] (biological process) Relationships: is a type of GO:0051324; BFO_0000050 mitotic M phase [GO:0000087] Note: Note that this term should not be used for direct annotation. If you are trying to make an annotation to x phase, it is likely that the correct annotation is 'regulation of x/y phase transition' or to a process which occurs during the reported phase (i.e mitotic DNA replication for mitotic S-phase). To capture the phase when a specific location or process is observed, the phase term can be used in an annotation extension (PMID:24885854) applied to a cellular component term (with the relation exists_during) or a biological process term (with the relation happens_during). Sources: GOC:mtg_cell_cycle Definition: The cell cycle phase which is the first stage of M phase of mitosis and during which chromosomes condense and the two daughter centrioles and their asters migrate toward the poles of the cell.